negative regulation of rDNA heterochromatin formation [GO:0061188] (biological process) Relationships: is a type of negative regulation of heterochromatin formation [GO:0031452]; is_a GO:0061187; negatively regulates GO:0000183 Also known as: negative regulation of chromatin silencing at rDNA, negative regulation of ribosomal DNA heterochromatin assembly, negative regulation of ribosomal DNA heterochromatin formation References: PMID:10388812 Sources: GOC:dph Definition: Any process that decreases the rate, frequency, or extent of ribosomal DNA heterochromatin formation.